{
  "term_id": "GO:0032281",
  "gene": "UniProtKB:Q9UF02",
  "term_label": "AMPA glutamate receptor complex",
  "gene_name": "Voltage-dependent calcium channel gamma-5 subunit",
  "gene_symbol": "CACNG5"
}